{
  "gene_symbol": "SEPTIN6",
  "gene_name": "Septin-6",
  "term_label": "molecular adaptor activity",
  "term_id": "GO:0060090",
  "gene": "UniProtKB:Q14141"
}